positive regulation of embryonic camera-type eye development [GO:1902865] (biological process) Definition: Any process that activates or increases the frequency, rate or extent of embryonic camera-type eye development. Also known as: positive regulation of embryonic eye development, up regulation of embryonic camera-type eye development, up regulation of embryonic eye development, up-regulation of embryonic camera-type eye development, up-regulation of embryonic eye development, upregulation of embryonic camera-type eye development, upregulation of embryonic eye development, activation of embryonic camera-type eye development, activation of embryonic eye development Relationships: is a type of positive regulation of developmental process [GO:0051094]; is a type of regulation of embryonic camera-type eye development [GO:1902863]; positively regulates embryonic camera-type eye development [GO:0031076] References: PMID:16872597 Sources: GOC:TermGenie, GOC:mr, GO_REF:0000058